{
  "term_label": "plasma membrane",
  "term_id": "GO:0005886",
  "gene_symbol": "MCHR1",
  "gene": "UniProtKB:Q99705",
  "gene_name": "Melanin-concentrating hormone receptor 1"
}